{
  "gene": "UniProtKB:Q8WVE0",
  "term_id": "GO:0016279",
  "term_label": "protein-lysine N-methyltransferase activity",
  "gene_symbol": "EEF1AKMT1",
  "gene_name": "EEF1A lysine methyltransferase 1"
}